{
  "gene": "UniProtKB:Q8N4V1",
  "term_id": "UNKNOWN:0002",
  "gene_symbol": "MMGT1",
  "term_label": "Unknown biological process",
  "gene_name": "ER membrane protein complex subunit 5"
}